{
  "gene": "UniProtKB:Q9UBU8",
  "gene_name": "Mortality factor 4-like protein 1",
  "term_label": "Unknown molecular function",
  "gene_symbol": "MORF4L1",
  "term_id": "UNKNOWN:0001"
}